{
  "term_id": "GO:0005615",
  "gene_symbol": "IFNA1",
  "gene": "UniProtKB:P01562",
  "term_label": "extracellular space",
  "gene_name": "Interferon alpha-1_13"
}